{
  "term_id": "GO:0007155",
  "term_label": "cell adhesion",
  "gene": "UniProtKB:Q9UMF0",
  "gene_name": "Intercellular adhesion molecule 5",
  "gene_symbol": "ICAM5"
}